myosin complex [GO:0016459] (cellular component) Subtypes: myosin II complex [GO:0016460], GO:0016461, actomyosin, myosin complex part [GO:0042642] Relationships: is a type of protein-containing complex [GO:0032991]; is part of actin cytoskeleton [GO:0015629] Definition: A protein complex, formed of one or more myosin heavy chains plus associated light chains and other proteins, that functions as a molecular motor; uses the energy of ATP hydrolysis to move actin filaments or to move vesicles or other cargo on fixed actin filaments; has magnesium-ATPase activity and binds actin. Myosin classes are distinguished based on sequence features of the motor, or head, domain, but also have distinct tail regions that are believed to bind specific cargoes. Sources: GOC:mah, Wikipedia:Myosin